{
  "gene": "UniProtKB:P19338",
  "term_id": "GO:0048027",
  "gene_symbol": "NCL",
  "term_label": "mRNA 5'-UTR binding",
  "gene_name": "Nucleolin"
}